cAMP-dependent protein kinase activity [GO:0004691] (molecular function) References: PMID:32935175, PMID:35053423, PMID:35805104 Also known as: protein kinase A activity, 3',5' cAMP-dependent protein kinase activity, 3',5'-cAMP-dependent protein kinase activity, adenosine 3',5'-cyclophosphate-dependent protein kinase activity, cAMP-dependent protein kinase, intrinsic catalyst activity, cyclic AMP-dependent protein kinase activity, AMPK, ATP:protein phosphotransferase (cAMP-dependent) activity, PKA, PKA C, STK22 Relationships: is a type of cyclic nucleotide-dependent protein kinase activity [GO:0004690]; has part cAMP binding [GO:0030552] Regulation: negatively regulated by cAMP-dependent protein kinase inhibitor activity [GO:0004862]; regulated by cAMP-dependent protein kinase regulator activity [GO:0008603]; regulated by GO:2000479; negatively regulated by GO:2000480; positively regulated by GO:2000481 Definition: cAMP-dependent catalysis of the reaction: ATP + a protein = ADP + a phosphoprotein. Note: This reaction requires the presence of cAMP.